{
  "term_label": "retrograde vesicle-mediated transport, Golgi to endoplasmic reticulum",
  "gene_symbol": "GOLPH3L",
  "gene_name": "Golgi phosphoprotein 3-like",
  "term_id": "GO:0006890",
  "gene": "UniProtKB:Q9H4A5"
}